{
  "term_id": "GO:0048665",
  "term_label": "neuron fate specification",
  "gene_name": "Insulin gene enhancer protein ISL-1",
  "gene": "UniProtKB:P61371",
  "gene_symbol": "ISL1"
}